allatostatin receptor activity [GO:0008261] (molecular function) Definition: Combining with allatostatin to initiate a change in cell activity. Relationships: is a type of GO:0008528 Sources: GOC:ai